{
  "gene": "UniProtKB:P21941",
  "gene_symbol": "MATN1",
  "term_id": "UNKNOWN:0001",
  "gene_name": "Cartilage matrix protein",
  "term_label": "Unknown molecular function"
}